{
  "term_id": "UNKNOWN:0001",
  "term_label": "Unknown molecular function",
  "gene_symbol": "BNIPL",
  "gene": "UniProtKB:Q7Z465",
  "gene_name": "Bcl-2_adenovirus E1B 19 kDa-interacting protein 2-like protein"
}